{
  "gene_name": "RIMS-binding protein 3A",
  "gene": "UniProtKB:Q9UFD9",
  "term_label": "nucleus",
  "term_id": "GO:0005634",
  "gene_symbol": "RIMBP3"
}